{
  "term_id": "GO:0038047",
  "gene_name": "Mu-type opioid receptor",
  "gene": "UniProtKB:P35372",
  "gene_symbol": "OPRM1",
  "term_label": "morphine receptor activity"
}